{
  "term_label": "cytoplasm",
  "gene_name": "PRAME family member 11",
  "gene_symbol": "PRAMEF11",
  "term_id": "GO:0005737",
  "gene": "UniProtKB:O60813"
}